{
  "gene_symbol": "FBXO22",
  "gene_name": "F-box only protein 22",
  "gene": "UniProtKB:Q8NEZ5",
  "term_id": "GO:0000209",
  "term_label": "protein polyubiquitination"
}